{
  "term_id": "UNKNOWN:0003",
  "gene_symbol": "LRRC49",
  "gene": "UniProtKB:Q8IUZ0",
  "gene_name": "Leucine-rich repeat-containing protein 49",
  "term_label": "Unknown cellular component"
}